{
  "term_label": "protein O-acetylglucosaminyltransferase activity",
  "gene_name": "UDP-N-acetylglucosamine--peptide N-acetylglucosaminyltransferase 110 kDa subunit",
  "gene_symbol": "OGT",
  "term_id": "GO:0097363",
  "gene": "UniProtKB:O15294"
}